{
  "gene_name": "TBC1 domain family member 25",
  "gene": "UniProtKB:Q3MII6",
  "gene_symbol": "TBC1D25",
  "term_label": "autophagosome",
  "term_id": "GO:0005776"
}